{
  "gene": "UniProtKB:Q8WTS1",
  "term_label": "lipid homeostasis",
  "gene_symbol": "ABHD5",
  "gene_name": "1-acylglycerol-3-phosphate O-acyltransferase ABHD5",
  "term_id": "GO:0055088"
}